{
  "term_label": "double-strand break repair",
  "gene_symbol": "MPND",
  "term_id": "GO:0006302",
  "gene_name": "MPN domain-containing protein",
  "gene": "UniProtKB:Q8N594"
}